{
  "term_id": "GO:0034359",
  "term_label": "mature chylomicron",
  "gene": "UniProtKB:P04114",
  "gene_symbol": "APOB",
  "gene_name": "Apolipoprotein B-100"
}